{
  "gene_name": "Serine_threonine-protein kinase A-Raf",
  "term_label": "MAP kinase kinase kinase activity",
  "term_id": "GO:0004709",
  "gene": "UniProtKB:P10398",
  "gene_symbol": "ARAF"
}